{
  "term_label": "DNA-binding transcription factor activity, RNA polymerase II-specific",
  "gene": "UniProtKB:O95343",
  "gene_name": "Homeobox protein SIX3",
  "gene_symbol": "SIX3",
  "term_id": "GO:0000981"
}